{
  "gene_symbol": "ARHGAP32",
  "term_label": "postsynaptic density",
  "gene_name": "Rho GTPase-activating protein 32",
  "gene": "UniProtKB:A7KAX9",
  "term_id": "GO:0014069"
}